{
  "term_label": "dopamine neurotransmitter receptor activity, coupled via Gs",
  "gene": "UniProtKB:P21918",
  "gene_name": "D(1B) dopamine receptor",
  "term_id": "GO:0001588",
  "gene_symbol": "DRD5"
}